{
  "term_id": "GO:0008307",
  "gene": "UniProtKB:O15273",
  "term_label": "structural constituent of muscle",
  "gene_name": "Telethonin",
  "gene_symbol": "TCAP"
}